{
  "term_label": "adenylate cyclase-modulating G protein-coupled receptor signaling pathway",
  "term_id": "GO:0007188",
  "gene_symbol": "DRD4",
  "gene_name": "D(4) dopamine receptor",
  "gene": "UniProtKB:P21917"
}